{
  "term_label": "Unknown biological process",
  "term_id": "UNKNOWN:0002",
  "gene_name": "Golgin subfamily A member 6-like protein 25",
  "gene_symbol": "GOLGA6L25",
  "gene": "UniProtKB:P0DX01"
}